phenylalanyl-tRNA aminoacylation [GO:0006432] (biological process) Subtypes: mitochondrial phenylalanyl-tRNA aminoacylation [GO:0070156] Relationships: is a type of GO:0006418 Definition: The process of coupling phenylalanine to phenylalanyl-tRNA, catalyzed by phenylalanyl-tRNA synthetase. The phenylalanyl-tRNA synthetase is a class-II synthetase. However, unlike other class II enzymes, The activated amino acid is transferred to the 2'-OH group of a phenylalanine-accepting tRNA. The 2'-O-aminoacyl-tRNA will ultimately migrate to the 3' position via transesterification. Sources: GOC:mcc, ISBN:0716730510